{
  "gene_symbol": "NDUFB8",
  "gene_name": "NADH dehydrogenase [ubiquinone] 1 beta subcomplex subunit 8, mitochondrial",
  "gene": "UniProtKB:O95169",
  "term_id": "UNKNOWN:0001",
  "term_label": "Unknown molecular function"
}